cytokine production involved in inflammatory response [GO:0002534] (biological process) Regulation: regulated by regulation of cytokine production involved in inflammatory response [GO:1900015]; negatively regulated by negative regulation of cytokine production involved in inflammatory response [GO:1900016]; positively regulated by positive regulation of cytokine production involved in inflammatory response [GO:1900017] Relationships: is a type of GO:0001816; is_a production of molecular mediator involved in inflammatory response [GO:0002532] Also known as: cytokine production involved in acute inflammatory response Definition: The synthesis or release of a cytokine following a inflammatory stimulus as part of an inflammatory response, resulting in an increase in its intracellular or extracellular levels. Sources: GOC:add, ISBN:0781735149